pyridoxine 5'-phosphate synthase activity [GO:0033856] (molecular function) Definition: Catalysis of the reaction: 1-deoxy-D-xylulose 5-phosphate + 3-amino-2-oxopropyl phosphate = 2 H2O + H+ + phosphate + pyridoxine 5'-phosphate. Also known as: 1-deoxy-D-xylulose-5-phosphate:3-amino-2-oxopropyl phosphate 3-amino-2-oxopropyltransferase (phosphate-hydrolysing; cyclizing) activity, PNP synthase activity, pyridoxine 5-phosphate phospho lyase activity Sources: RHEA:15265 Relationships: is a type of GO:0016769